{
  "gene_name": "OTU domain-containing protein 5",
  "term_label": "regulation of immune response",
  "gene": "UniProtKB:Q96G74",
  "term_id": "GO:0050776",
  "gene_symbol": "OTUD5"
}